{
  "gene": "UniProtKB:P21579",
  "gene_name": "Synaptotagmin-1",
  "gene_symbol": "SYT1",
  "term_id": "GO:0005544",
  "term_label": "calcium-dependent phospholipid binding"
}